regulation of gastrulation [GO:0010470] (biological process) Definition: Any process that modulates the rate or extent of gastrulation. Gastrulation is the complex and coordinated series of cellular movements that occurs at the end of cleavage during embryonic development of most animals. Sources: GOC:dph, GOC:tb Relationships: is a type of regulation of anatomical structure morphogenesis [GO:0022603]; is a type of GO:0045995; regulates gastrulation [GO:0007369] Subtypes: GO:0110073, negative regulation of gastrulation [GO:2000542], positive regulation of gastrulation [GO:2000543]